{
  "term_label": "Unknown cellular component",
  "gene": "UniProtKB:P0DP04",
  "term_id": "UNKNOWN:0003",
  "gene_symbol": "IGHV3-43D",
  "gene_name": "Immunoglobulin heavy variable 3-43D"
}